{
  "gene_name": "Protein MTO1 homolog, mitochondrial",
  "term_id": "GO:0005739",
  "term_label": "mitochondrion",
  "gene_symbol": "MTO1",
  "gene": "UniProtKB:Q9Y2Z2"
}